{
  "term_id": "UNKNOWN:0002",
  "gene": "UniProtKB:Q96DL1",
  "gene_name": "NXPE family member 2",
  "gene_symbol": "NXPE2",
  "term_label": "Unknown biological process"
}